{
  "gene": "UniProtKB:Q9HD89",
  "gene_symbol": "RETN",
  "gene_name": "Resistin",
  "term_id": "UNKNOWN:0002",
  "term_label": "Unknown biological process"
}